{
  "gene_name": "Fas-activated serine_threonine kinase",
  "gene": "UniProtKB:Q14296",
  "term_id": "GO:0000963",
  "gene_symbol": "FASTK",
  "term_label": "mitochondrial RNA processing"
}